{
  "gene_symbol": "CHN1",
  "gene": "UniProtKB:P15882",
  "gene_name": "N-chimaerin",
  "term_label": "ephrin receptor binding",
  "term_id": "GO:0046875"
}